indole-3-acetyl-isoleucine synthetase activity [GO:0102048] (molecular function) Definition: Catalysis of the reaction: indole-3-acetate + L-isoleucine + ATP(4-) = H+ + indole-3-acetyl-isoleucine + AMP(2-) + diphosphoric acid. References: PMID:15659623 Sources: GOC:pz Relationships: is a type of ligase activity, forming carbon-nitrogen bonds [GO:0016879]